{
  "gene_name": "Myosin-binding protein C, cardiac-type",
  "term_label": "ventricular cardiac muscle tissue morphogenesis",
  "gene": "UniProtKB:Q14896",
  "term_id": "GO:0055010",
  "gene_symbol": "MYBPC3"
}